anestrus phase [GO:0160266] (biological process) Definition: A biological phase of reproductive dormancy characterized by the temporary cessation of reproductive cyclicity, marked by the absence of ovarian follicular development, estrous behavior, and ovulation. This phase represents a period of sexual quiescence between estrous cycles or breeding seasons. Note: Note that this term should not be used for direct annotation. If you are trying to make an annotation to x phase, it is likely that the correct annotation is 'regulation of x/y phase transition' or to a process which occurs during the reported phase. To capture the phase when a specific location or process is observed, the phase term can be used in an annotation extension (PMID:24885854) applied to a cellular component term (with the relation exists_during) or a biological process term (with the relation happens_during). References: PMID:34635709 Sources: WIKIPEDIA:Estrous_cycle Relationships: is a type of biological phase [GO:0044848]